{
  "term_label": "cytoplasm",
  "term_id": "GO:0005737",
  "gene_symbol": "FRAT2",
  "gene": "UniProtKB:O75474",
  "gene_name": "GSK-3-binding protein FRAT2"
}